{
  "term_id": "UNKNOWN:0001",
  "gene": "UniProtKB:P11532",
  "gene_symbol": "DMD",
  "gene_name": "Dystrophin",
  "term_label": "Unknown molecular function"
}